{
  "gene_name": "Gigaxonin",
  "term_id": "GO:0031463",
  "gene": "UniProtKB:Q9H2C0",
  "gene_symbol": "GAN",
  "term_label": "Cul3-RING ubiquitin ligase complex"
}